{
  "term_label": "Unknown molecular function",
  "term_id": "UNKNOWN:0001",
  "gene_symbol": "CTSL3P",
  "gene_name": "Putative inactive cathepsin L-like protein CTSL3P",
  "gene": "UniProtKB:Q5NE16"
}